photoreceptor inner segment [GO:0001917] (cellular component) Relationships: is a type of GO:0110165 References: PMID:12019563 Sources: GOC:add Definition: The inner segment of a vertebrate photoreceptor containing mitochondria, ribosomes and membranes where opsin molecules are assembled and passed to be part of the outer segment discs.